regulation of interleukin-15 production [GO:0032658] (biological process) Sources: GOC:mah Definition: Any process that modulates the frequency, rate, or extent of interleukin-15 production. Subtypes: negative regulation of interleukin-15 production [GO:0032698], GO:0032738 Relationships: is a type of regulation of cytokine production [GO:0001817]; regulates interleukin-15 production [GO:0032618] Also known as: regulation of IL-15 production, regulation of interleukin-15 biosynthetic process